{
  "gene_name": "Zinc finger protein 133",
  "gene_symbol": "ZNF133",
  "gene": "UniProtKB:P52736",
  "term_id": "GO:0000981",
  "term_label": "DNA-binding transcription factor activity, RNA polymerase II-specific"
}